{
  "gene": "UniProtKB:Q68CZ2",
  "term_id": "GO:0035022",
  "term_label": "positive regulation of Rac protein signal transduction",
  "gene_symbol": "TNS3",
  "gene_name": "Tensin-3"
}